{
  "gene_name": "Stromal interaction molecule 1",
  "term_id": "GO:0002115",
  "term_label": "store-operated calcium entry",
  "gene_symbol": "STIM1",
  "gene": "UniProtKB:Q13586"
}